{
  "term_id": "GO:0140285",
  "gene_name": "WASH complex subunit 5",
  "gene_symbol": "WASHC5",
  "gene": "UniProtKB:Q12768",
  "term_label": "endosome fission"
}